orotate phosphoribosyltransferase activity [GO:0004588] (molecular function) Relationships: is a type of pentosyltransferase activity [GO:0016763] Also known as: OPRT activity, OPRTase activity, orotate phosphoribosyl pyrophosphate transferase activity, orotic acid phosphoribosyltransferase activity, orotidine 5'-monophosphate pyrophosphorylase activity, orotidine monophosphate pyrophosphorylase activity, orotidine phosphoribosyltransferase activity, orotidine-5'-phosphate diphosphorylase activity, orotidine-5'-phosphate pyrophosphorylase activity, orotidine-5'-phosphate:diphosphate phospho-alpha-D-ribosyl-transferase activity, orotidylate phosphoribosyltransferase activity, orotidylate pyrophosphorylase activity, orotidylic acid phosphorylase activity, orotidylic acid pyrophosphorylase activity, orotidylic phosphorylase activity, orotidylic pyrophosphorylase activity Definition: Catalysis of the reaction: orotidine 5'-phosphate + diphosphate = orotate + 5-phospho-alpha-D-ribose 1-diphosphate. Sources: EC:2.4.2.10